regulation of meristem development [GO:0048509] (BP) Sources: GOC:jid Subtypes: regulation of timing of meristematic phase transition [GO:0048506], regulation of shoot apical meristem development [GO:1902183] Relationships: is a type of regulation of developmental process [GO:0050793]; RO_0002211 GO:0048507 Definition: Any process that modulates the frequency, rate or extent of meristem development, the biological process whose specific outcome is the progression of the meristem over time, from its formation to the mature structure.